{
  "gene": "UniProtKB:P01584",
  "term_label": "regulation of ERK1 and ERK2 cascade",
  "term_id": "GO:0070372",
  "gene_symbol": "IL1B",
  "gene_name": "Interleukin-1 beta"
}